{
  "gene": "UniProtKB:Q96FN5",
  "term_label": "microtubule",
  "gene_symbol": "KIF12",
  "gene_name": "Kinesin-like protein KIF12",
  "term_id": "GO:0005874"
}